{
  "gene": "UniProtKB:A6NHR9",
  "gene_symbol": "SMCHD1",
  "term_label": "Unknown molecular function",
  "gene_name": "Structural maintenance of chromosomes flexible hinge domain-containing protein 1",
  "term_id": "UNKNOWN:0001"
}